{
  "gene_symbol": "UVRAG",
  "gene_name": "UV radiation resistance-associated gene protein",
  "gene": "UniProtKB:Q9P2Y5",
  "term_label": "lytic vacuole",
  "term_id": "GO:0000323"
}